{
  "term_id": "GO:0005737",
  "term_label": "cytoplasm",
  "gene_symbol": "PYGB",
  "gene": "UniProtKB:P11216",
  "gene_name": "Glycogen phosphorylase, brain form"
}